{
  "gene_name": "Zinc finger protein 607",
  "gene": "UniProtKB:Q96SK3",
  "term_id": "GO:0000978",
  "term_label": "RNA polymerase II cis-regulatory region sequence-specific DNA binding",
  "gene_symbol": "ZNF607"
}